{
  "term_id": "GO:0007005",
  "gene_symbol": "STOML2",
  "gene_name": "Stomatin-like protein 2, mitochondrial",
  "term_label": "mitochondrion organization",
  "gene": "UniProtKB:Q9UJZ1"
}